negative regulation of leucine import in response to ammonium ion [GO:0060360] (biological process) Definition: Any process that decreases the rate, frequency or extent of leucine import as a result of an ammonium ion stimulus. Leucine import is the directed movement of leucine into a cell or organelle. Also known as: negative regulation of leucine uptake in response to ammonium ion Relationships: is a type of negative regulation of L-leucine import across plasma membrane [GO:1905533]; BFO_0000050 cellular response to ammonium ion [GO:0071242] Sources: GOC:dph, GOC:tb